behavioral response to formalin induced pain [GO:0061368] (biological process) Definition: Any process that results in a change in the behaviour of an organism as a result of a formalin pain stimulus. Relationships: is a type of GO:0061366 Sources: GOC:dph